{
  "term_id": "UNKNOWN:0002",
  "gene": "UniProtKB:Q5VW22",
  "term_label": "Unknown biological process",
  "gene_symbol": "AGAP6",
  "gene_name": "Arf-GAP with GTPase, ANK repeat and PH domain-containing protein 6"
}